negative regulation of intrinsic apoptotic signaling pathway by p53 class mediator [GO:1902254] (biological process) Also known as: down regulation of intrinsic apoptotic signaling pathway by p53 class mediator, down regulation of intrinsic apoptotic signaling pathway by signal transduction by p53 class mediator, down-regulation of intrinsic apoptotic signaling pathway by p53 class mediator, down-regulation of intrinsic apoptotic signaling pathway by signal transduction by p53 class mediator, downregulation of intrinsic apoptotic signaling pathway by p53 class mediator, downregulation of intrinsic apoptotic signaling pathway by signal transduction by p53 class mediator, negative regulation of intrinsic apoptotic signaling pathway by signal transduction by p53 class mediator, inhibition of intrinsic apoptotic signaling pathway by p53 class mediator, inhibition of intrinsic apoptotic signaling pathway by signal transduction by p53 class mediator, down regulation of signal transduction by p53 class mediator resulting in induction of apoptosis, down-regulation of signal transduction by p53 class mediator resulting in induction of apoptosis, downregulation of signal transduction by p53 class mediator resulting in induction of apoptosis, inhibition of signal transduction by p53 class mediator resulting in induction of apoptosis, negative regulation of signal transduction by p53 class mediator resulting in induction of apoptosis Definition: Any process that stops, prevents or reduces the frequency, rate or extent of intrinsic apoptotic signaling pathway by p53 class mediator. Subtypes: negative regulation of intrinsic apoptotic signaling pathway in response to DNA damage by p53 class mediator [GO:1902166], negative regulation of intrinsic apoptotic signaling pathway in response to osmotic stress by p53 class mediator [GO:1902239] Relationships: is a type of negative regulation of signal transduction by p53 class mediator [GO:1901797]; is a type of regulation of intrinsic apoptotic signaling pathway by p53 class mediator [GO:1902253]; is a type of negative regulation of intrinsic apoptotic signaling pathway [GO:2001243]; negatively regulates intrinsic apoptotic signaling pathway by p53 class mediator [GO:0072332] References: PMID:15705871 Sources: GOC:BHF, GOC:TermGenie, GOC:mtg_apoptosis, GOC:rl